{
  "term_label": "protein K11-linked ubiquitination",
  "gene_symbol": "UBE2L5",
  "gene": "UniProtKB:A0A1B0GUS4",
  "term_id": "GO:0070979",
  "gene_name": "Ubiquitin-conjugating enzyme E2 L5"
}